{
  "term_id": "GO:0004674",
  "gene_name": "Serine_threonine-protein kinase MRCK alpha",
  "gene_symbol": "CDC42BPA",
  "term_label": "protein serine/threonine kinase activity",
  "gene": "UniProtKB:Q5VT25"
}